{
  "gene_name": "Transforming growth factor beta-1-induced transcript 1 protein",
  "term_label": "Unknown molecular function",
  "gene": "UniProtKB:O43294",
  "term_id": "UNKNOWN:0001",
  "gene_symbol": "TGFB1I1"
}